DNA strand elongation [GO:0022616] (biological process) Definition: The DNA metabolic process in which an existing DNA strand is extended by activities including the addition of nucleotides to the 3' end of the strand. Sources: GOC:isa_complete, GOC:mah Relationships: is a type of DNA metabolic process [GO:0006259]; has part GO:0071897 Subtypes: DNA strand elongation involved in DNA replication [GO:0006271], telomeric 3' overhang formation [GO:0031860] Regulation: regulated by regulation of DNA strand elongation [GO:0060382]; positively regulated by positive regulation of DNA strand elongation [GO:0060383]